{
  "term_label": "immune response",
  "gene_symbol": "IGLV3-16",
  "gene_name": "Immunoglobulin lambda variable 3-16",
  "term_id": "GO:0006955",
  "gene": "UniProtKB:A0A075B6K0"
}